oxalate:chloride antiporter activity [GO:0160046] (molecular function) References: PMID:17442754 Relationships: is a type of GO:0005452; is a type of GO:0015108; is a type of oxalate transmembrane transporter activity [GO:0019531] Definition: Enables the transfer of a solute or solutes from one side of a membrane to the other according to the reaction: chloride(out) + oxalate(in) = chloride(in) + oxalate(out).